{
  "gene_symbol": "RHOJ",
  "gene": "UniProtKB:Q9H4E5",
  "term_label": "plasma membrane",
  "gene_name": "Rho-related GTP-binding protein RhoJ",
  "term_id": "GO:0005886"
}